{
  "term_id": "GO:0006309",
  "gene_name": "Endonuclease G, mitochondrial",
  "gene": "UniProtKB:Q14249",
  "term_label": "apoptotic DNA fragmentation",
  "gene_symbol": "ENDOG"
}